molecular sequestering activity [GO:0140313] (molecular function) Subtypes: toxin sequestering activity [GO:0097351], protein sequestering activity [GO:0140311], receptor decoy activity [GO:0140319], metal ion sequestering activity [GO:0140487], GO:0140610 Definition: Binding to a specific molecule to prevent it from interacting with other partners or to inhibit its localization to the area of the cell or complex where it is active. Relationships: is a type of molecular_function [GO:0003674] References: PMID:13130076